{
  "term_label": "RNA polymerase II cis-regulatory region sequence-specific DNA binding",
  "gene_symbol": "ZNF527",
  "term_id": "GO:0000978",
  "gene": "UniProtKB:Q8NB42",
  "gene_name": "Zinc finger protein 527"
}